acetoacetic acid metabolic process [GO:0043438] (biological process) Sources: Wikipedia:Acetoacetic_acid Relationships: is a type of short-chain fatty acid metabolic process [GO:0046459]; is a type of GO:1902224 Also known as: 3-oxobutanoate metabolic process, 3-oxobutanoate metabolism, 3-oxobutanoic acid metabolic process, 3-oxobutanoic acid metabolism, acetoacetate metabolic process, acetoacetate metabolism, acetoacetic acid metabolism, beta ketobutyric acid metabolic process, beta ketobutyric acid metabolism, beta-ketobutyric acid metabolic process, beta-ketobutyric acid metabolism, diacetic acid metabolic process, diacetic acid metabolism Subtypes: GO:0043441, GO:0043442 Definition: The chemical reactions and pathways involving acetoacetic acid, 3-oxobutanoic acid; the empirical formula is C4H6O3 or CH3COCH2COOH.